{
  "gene_symbol": "KCTD12",
  "term_label": "postsynaptic membrane",
  "term_id": "GO:0045211",
  "gene": "UniProtKB:Q96CX2",
  "gene_name": "BTB_POZ domain-containing protein KCTD12"
}